{
  "term_id": "UNKNOWN:0002",
  "gene_symbol": "NENF",
  "gene_name": "Neudesin",
  "gene": "UniProtKB:Q9UMX5",
  "term_label": "Unknown biological process"
}